positive regulation of formation by symbiont of haustorium for nutrient acquisition from host [GO:0075046] (biological process) Sources: GOC:pamgo_curators Note: Note that this term should not be used to annotate gene products of the host. It should only be used to annotate those gene products from the symbiont involved in this process. Relationships: is a type of positive regulation of formation of structure involved in a symbiotic process [GO:0044149]; is a type of regulation of formation by symbiont of haustorium for nutrient acquisition from host [GO:0075045]; positively regulates GO:0052094 Definition: Any process that activates or increases the frequency, rate or extent of symbiont haustorium formation for nutrient acquisition from host. The host is defined as the larger of the organisms involved in a symbiotic interaction.